{
  "gene_name": "Syndecan-4",
  "term_label": "Unknown molecular function",
  "gene": "UniProtKB:P31431",
  "term_id": "UNKNOWN:0001",
  "gene_symbol": "SDC4"
}